{
  "gene": "UniProtKB:Q8IYX0",
  "term_label": "Unknown cellular component",
  "term_id": "UNKNOWN:0003",
  "gene_name": "Zinc finger protein 679",
  "gene_symbol": "ZNF679"
}